{
  "term_label": "poly(A)+ mRNA export from nucleus",
  "gene_name": "Transcription and mRNA export factor ENY2",
  "gene_symbol": "ENY2",
  "gene": "UniProtKB:Q9NPA8",
  "term_id": "GO:0016973"
}